{
  "gene": "UniProtKB:Q8N1F7",
  "gene_symbol": "NUP93",
  "term_id": "GO:0006606",
  "gene_name": "Nuclear pore complex protein Nup93",
  "term_label": "protein import into nucleus"
}